acetyl-CoA binding [GO:1905502] (MF) Relationships: is a type of acyl-CoA binding [GO:0120227] References: PMID:24927529 Sources: GOC:PARL, GOC:TermGenie, GOC:bc, GOC:krc, GO_REF:0000067 Also known as: acetyl-coenzyme A binding Definition: Binding to acetyl-CoA, an acyl-CoA having acetyl as its S-acetyl component.